{
  "term_id": "GO:0016342",
  "gene_symbol": "CDH26",
  "term_label": "catenin complex",
  "gene": "UniProtKB:Q8IXH8",
  "gene_name": "Cadherin-like protein 26"
}